yolk granule [GO:0042718] (cellular component) Definition: Discrete structures that partition the water-insoluble portion of the yolk of oocytes and ova, which may or may not be membrane enclosed. Relationships: is a type of GO:0110165; is part of yolk [GO:0060417] References: PMID:18046696, PMID:6337890 Sources: GOC:jl